{
  "term_label": "malate metabolic process",
  "term_id": "GO:0006108",
  "gene_symbol": "ME2",
  "gene": "UniProtKB:P23368",
  "gene_name": "NAD-dependent malic enzyme, mitochondrial"
}